contractile vacuole complex [GO:0062159] (CC) Relationships: is a type of GO:0043232 References: PMID:23890380 Definition: A non-membrane-bounded organelle of eukaryotic cells, especially Protozoa, that fills with water from the cytoplasm and then discharges this externally. One of its functions is osmoregulatory. Also known as: CVC